D-gluconate biosynthetic process [GO:0046178] (biological process) Sources: ISBN:0198506732 Relationships: is a type of carbohydrate biosynthetic process [GO:0016051]; is a type of D-gluconate metabolic process [GO:0019521]; is a type of GO:0046175 Definition: The chemical reactions and pathways resulting in the formation of D-gluconate, the anion of D-gluconic acid, the aldonic acid derived from glucose. Also known as: D-gluconate anabolism, D-gluconate biosynthesis, D-gluconate formation, D-gluconate synthesis